'de novo' NAD+ biosynthetic process from L-tryptophan [GO:0034354] (biological process) Definition: The chemical reactions and pathways resulting in the formation of nicotinamide adenine dinucleotide (NAD+), beginning with the catabolism of L-tryptophan into the precursor quinolinate. NAD+ is a coenzyme that interconverts with its reduced form, NADH, in many redox and catabolic reactions. References: PMID:17161604 Also known as: 'de novo' NAD biosynthetic process from tryptophan, 'de novo' NAD biosynthetic process from L-tryptophan, de novo NAD biosynthetic process from tryptophan Regulation: regulated by regulation of 'de novo' NAD biosynthetic process from L-tryptophan [GO:1905012]; negatively regulated by negative regulation of 'de novo' NAD biosynthetic process from L-tryptophan [GO:1905013]; RO_0002213 by GO:1905014 Relationships: is a type of L-tryptophan metabolic process [GO:0006568]; is a type of NAD+ biosynthetic process [GO:0009435]